regulation of sporocarp development involved in sexual reproduction [GO:1902058] (biological process) Subtypes: regulation of cleistothecium development [GO:0070796], GO:1902059, positive regulation of sporocarp development involved in sexual reproduction [GO:1902060] Definition: Any process that modulates the frequency, rate or extent of sporocarp development involved in sexual reproduction. Also known as: regulation of fruiting body development involved in sexual reproduction, regulation of fruiting body formation involved in sexual reproduction, regulation of ascus development, regulation of perfect stage fruiting body development Relationships: is a type of regulation of reproductive fruiting body development [GO:0031155]; regulates sporocarp development involved in sexual reproduction [GO:0000909] References: PMID:23480775 Sources: GOC:TermGenie, GOC:di